siRNA-mediated heterochromatin formation [GO:0141194] (biological process) Relationships: is a type of regulatory ncRNA-mediated heterochromatin formation [GO:0031048] Subtypes: GO:0080188, siRNA-mediated silent mating type cassette region heterochromatin formation [GO:0140185], siRNA-mediated pericentric heterochromatin formation [GO:0140727], transposable element silencing by siRNA-mediated heterochromatin formation [GO:0141007], siRNA-mediated facultative heterochromatin formation [GO:1902795] Definition: The formation of heterochromatin into a heterochromatin domain by a process mediated by a small interfering siRNA. Sources: GOC:ha, GOC:pg